{
  "gene_name": "Histone H3.Y",
  "term_id": "GO:0031492",
  "term_label": "nucleosomal DNA binding",
  "gene": "UniProtKB:P0DPK2",
  "gene_symbol": "H3Y1"
}